{
  "term_id": "UNKNOWN:0003",
  "gene_name": "Pyridine nucleotide-disulfide oxidoreductase domain-containing protein 2",
  "term_label": "Unknown cellular component",
  "gene": "UniProtKB:Q8N2H3",
  "gene_symbol": "PYROXD2"
}